{
  "term_label": "Unknown molecular function",
  "gene_name": "Cysteine-rich hydrophobic domain-containing protein 1",
  "gene_symbol": "CHIC1",
  "term_id": "UNKNOWN:0001",
  "gene": "UniProtKB:Q5VXU3"
}